purine ribonucleotide interconversion [GO:0015951] (BP) Sources: GOC:mah, ISBN:0306444747, ISBN:0471394831 Definition: The chemical reactions and pathways by which a purine ribonucleotide is synthesized from another purine ribonucleotide. Relationships: is a type of purine ribonucleotide metabolic process [GO:0009150]; is a type of purine nucleotide interconversion [GO:0015950]